regulation of vitamin D biosynthetic process [GO:0060556] (biological process) Relationships: is a type of regulation of vitamin metabolic process [GO:0030656]; is a type of GO:0050810; regulates vitamin D biosynthetic process [GO:0042368] Sources: CHEBI:27300, GOC:BHF, GOC:mah, ISBN:0471331309 Definition: Any process that modulates the rate frequency or extent of a vitamin D biosynthetic process. Vitamin D biosynthesis is the chemical reactions and pathways resulting in the formation of vitamin D, any of a group of related, fat-soluble compounds that are derived from delta-5,7 steroids and play a central role in calcium metabolism. Specific forms of vitamin D include calciferol (ergocalciferol; vitamin D2) and cholecalciferol (calciol; vitamin D3). Subtypes: negative regulation of vitamin D biosynthetic process [GO:0010957], positive regulation of vitamin D biosynthetic process [GO:0060557]